cytosolic ciliogenesis [GO:0061824] (biological process) Also known as: intracellular ciliogenesis Definition: The process in which an axoneme is exposed entirely or partially to the cytoplasm or by which the cytoplasmic portion is assembled or extended. Cytosolic ciliogenesis can occur following compartmentalized ciliogenesis, in which the cilium is formed within a compartment separated from the cytoplasm. References: PMID:25447994, PMID:26654377 Relationships: is a type of GO:0060271